corrinoid adenosyltransferase activity [GO:0008817] (molecular function) Definition: Catalysis of the reaction: 2 ATP + 2 corrinoid + reduced [electron-transfer flavoprotein] = 2 adenosylcorrinoid + 3 H+ + oxidized [electron-transfer flavoprotein] + 2 triphosphate. The corrinoid can be cob(II)yrinate a,c diamide, cob(II)inamide or cob(II)alamin. Also known as: ATP:cob(I)alamin Co-beta-adenosyltransferase activity, ATP:cob(I)yrinic acid-a,c-diamide cobeta-adenosyltransferase activity, aquacob(I)alamin adenosyltransferase activity, aquocob(I)alamin vitamin B12s adenosyltransferase activity, cob(I)alamin adenosyltransferase activity, cob(I)yrinic acid a,c-diamide adenosyltransferase activity, cob(II)yrinic acid a,c-diamide reductase activity, cob(II)yrinic acid-a,c-diamide:FMN oxidoreductase activity, ATP:cob(I)alamin cobeta-adenosyltransferase activity, ATP:corrinoid adenosyltransferase activity, vitamin B12s adenosyltransferase activity Relationships: is a type of GO:0016765 References: PMID:19933577, PMID:5946606